{
  "term_label": "stereocilium tip",
  "gene": "UniProtKB:Q9H5P4",
  "gene_name": "PDZ domain-containing protein 7",
  "term_id": "GO:0032426",
  "gene_symbol": "PDZD7"
}